{
  "gene_symbol": "ENGASE",
  "gene_name": "Cytosolic endo-beta-N-acetylglucosaminidase",
  "gene": "UniProtKB:Q8NFI3",
  "term_id": "GO:0033925",
  "term_label": "mannosyl-glycoprotein endo-beta-N-acetylglucosaminidase activity"
}